{
  "gene_symbol": "CCDC177",
  "term_label": "Unknown cellular component",
  "gene": "UniProtKB:Q9NQR7",
  "gene_name": "Coiled-coil domain-containing protein 177",
  "term_id": "UNKNOWN:0003"
}